{
  "term_id": "GO:0099184",
  "term_label": "structural constituent of postsynaptic intermediate filament cytoskeleton",
  "gene_name": "Neurofilament light polypeptide",
  "gene": "UniProtKB:P07196",
  "gene_symbol": "NEFL"
}